{
  "gene_name": "Histone lysine demethylase PHF8",
  "term_id": "GO:0006357",
  "gene": "UniProtKB:Q9UPP1",
  "term_label": "regulation of transcription by RNA polymerase II",
  "gene_symbol": "PHF8"
}